{
  "term_id": "GO:0045765",
  "gene_symbol": "VASH2",
  "term_label": "regulation of angiogenesis",
  "gene": "UniProtKB:Q86V25",
  "gene_name": "Tubulinyl-Tyr carboxypeptidase 2"
}